{
  "gene_name": "Stress-induced-phosphoprotein 1",
  "term_id": "UNKNOWN:0003",
  "gene_symbol": "STIP1",
  "term_label": "Unknown cellular component",
  "gene": "UniProtKB:P31948"
}